{
  "term_label": "regulation of cell population proliferation",
  "gene": "UniProtKB:Q6VUC0",
  "term_id": "GO:0042127",
  "gene_name": "Transcription factor AP-2-epsilon",
  "gene_symbol": "TFAP2E"
}